{
  "gene_symbol": "TAS1R2",
  "gene": "UniProtKB:Q8TE23",
  "term_id": "GO:0004930",
  "term_label": "G protein-coupled receptor activity",
  "gene_name": "Taste receptor type 1 member 2"
}